{
  "gene_name": "Extended synaptotagmin-2",
  "term_id": "GO:0005509",
  "term_label": "calcium ion binding",
  "gene_symbol": "ESYT2",
  "gene": "UniProtKB:A0FGR8"
}